{
  "gene_name": "Uncharacterized protein C2orf72",
  "gene_symbol": "C2orf72",
  "term_label": "Unknown molecular function",
  "gene": "UniProtKB:A6NCS6",
  "term_id": "UNKNOWN:0001"
}